gibberellin metabolic process [GO:0009685] (biological process) Subtypes: GO:0009686, GO:0045487 Definition: The chemical reactions and pathways involving gibberellin. Gibberellins are a class of highly modified terpenes that function as plant growth regulators. Relationships: is_a GO:0016101; is a type of GO:0019752 Also known as: gibberellin metabolism, gibberellic acid metabolic process, gibberellic acid metabolism Sources: ISBN:0387969845